{
  "gene": "UniProtKB:Q5T871",
  "term_id": "UNKNOWN:0002",
  "gene_name": "Late cornified envelope-like proline-rich protein 1",
  "gene_symbol": "LELP1",
  "term_label": "Unknown biological process"
}